{
  "term_id": "GO:0006357",
  "gene": "UniProtKB:P25440",
  "term_label": "regulation of transcription by RNA polymerase II",
  "gene_symbol": "BRD2",
  "gene_name": "Bromodomain-containing protein 2"
}